{
  "gene_name": "Putative RRN3-like protein RRN3P1",
  "term_label": "Unknown biological process",
  "term_id": "UNKNOWN:0002",
  "gene_symbol": "RRN3P1",
  "gene": "UniProtKB:Q2M238"
}